{
  "gene": "UniProtKB:Q5T5X7",
  "term_label": "rDNA heterochromatin formation",
  "term_id": "GO:0000183",
  "gene_symbol": "BEND3",
  "gene_name": "BEN domain-containing protein 3"
}